{
  "term_label": "beta1-adrenergic receptor activity",
  "gene_symbol": "ADRB1",
  "term_id": "GO:0004940",
  "gene": "UniProtKB:P08588",
  "gene_name": "Beta-1 adrenergic receptor"
}